{
  "term_label": "Unknown cellular component",
  "gene_name": "Bifunctional coenzyme A synthase",
  "term_id": "UNKNOWN:0003",
  "gene": "UniProtKB:Q13057",
  "gene_symbol": "COASY"
}